{
  "gene_name": "1-phosphatidylinositol 3-phosphate 5-kinase",
  "gene": "UniProtKB:Q9Y2I7",
  "term_id": "GO:0032438",
  "term_label": "melanosome organization",
  "gene_symbol": "PIKFYVE"
}